{
  "term_id": "GO:0043025",
  "gene_symbol": "STRN4",
  "gene": "UniProtKB:Q9NRL3",
  "gene_name": "Striatin-4",
  "term_label": "neuronal cell body"
}